{
  "term_id": "GO:0005886",
  "gene_symbol": "NTSR2",
  "term_label": "plasma membrane",
  "gene_name": "Neurotensin receptor type 2",
  "gene": "UniProtKB:O95665"
}